{
  "gene_name": "2'-5'-oligoadenylate synthase 1",
  "term_label": "2'-5'-oligoadenylate synthetase activity",
  "gene_symbol": "OAS1",
  "term_id": "GO:0001730",
  "gene": "UniProtKB:P00973"
}